{
  "term_id": "GO:0008270",
  "term_label": "zinc ion binding",
  "gene_symbol": "QPCTL",
  "gene": "UniProtKB:Q9NXS2",
  "gene_name": "Glutaminyl-peptide cyclotransferase-like protein"
}